{
  "term_id": "GO:0005811",
  "gene_name": "Perilipin-5",
  "gene_symbol": "PLIN5",
  "gene": "UniProtKB:Q00G26",
  "term_label": "lipid droplet"
}